{
  "gene_name": "Ankyrin repeat domain-containing protein 13C",
  "term_label": "protein targeting to membrane",
  "gene": "UniProtKB:Q8N6S4",
  "gene_symbol": "ANKRD13C",
  "term_id": "GO:0006612"
}